regulation of corticosterone secretion [GO:2000852] (biological process) Relationships: is_a regulation of glucocorticoid secretion [GO:2000849]; regulates corticosterone secretion [GO:0035934] Subtypes: GO:2000853, GO:2000854 Definition: Any process that modulates the frequency, rate or extent of corticosterone secretion. Sources: GOC:sl